apelin receptor activity [GO:0060182] (molecular function) Definition: Combining with the peptide apelin to initiate a change in cell activity. Sources: GOC:dph Relationships: is a type of G protein-coupled peptide receptor activity [GO:0008528]; is part of apelin receptor signaling pathway [GO:0060183]